{
  "term_label": "neuron migration",
  "gene_name": "Neogenin",
  "term_id": "GO:0001764",
  "gene": "UniProtKB:Q92859",
  "gene_symbol": "NEO1"
}